{
  "gene": "UniProtKB:Q6IEY1",
  "term_label": "olfactory receptor activity",
  "term_id": "GO:0004984",
  "gene_symbol": "OR4F16",
  "gene_name": "Olfactory receptor 4F3_4F16_4F29"
}